{
  "gene": "UniProtKB:Q9H2E6",
  "gene_symbol": "SEMA6A",
  "gene_name": "Semaphorin-6A",
  "term_id": "GO:0071526",
  "term_label": "semaphorin-plexin signaling pathway"
}